{
  "term_id": "GO:0005741",
  "gene_name": "Mitochondrial dynamics protein MID49",
  "gene_symbol": "MIEF2",
  "term_label": "mitochondrial outer membrane",
  "gene": "UniProtKB:Q96C03"
}